{
  "gene_symbol": "TM4SF19",
  "term_id": "UNKNOWN:0001",
  "gene_name": "Transmembrane 4 L6 family member 19",
  "term_label": "Unknown molecular function",
  "gene": "UniProtKB:Q96DZ7"
}